{
  "gene_name": "Glucose-6-phosphate 1-dehydrogenase",
  "gene": "UniProtKB:P11413",
  "term_id": "GO:0006006",
  "term_label": "glucose metabolic process",
  "gene_symbol": "G6PD"
}